{
  "gene_name": "Phospholipase A2, membrane associated",
  "gene": "UniProtKB:P14555",
  "term_label": "Unknown cellular component",
  "term_id": "UNKNOWN:0003",
  "gene_symbol": "PLA2G2A"
}